negative regulation of sebum secreting cell proliferation [GO:1904003] (biological process) Definition: Any process that stops, prevents or reduces the frequency, rate or extent of sebum secreting cell proliferation. References: PMID:16901790 Sources: GOC:TermGenie, GOC:hjd, GO_REF:0000058 Also known as: down regulation of sebum secreting cell proliferation, down-regulation of sebum secreting cell proliferation, downregulation of sebum secreting cell proliferation, inhibition of sebum secreting cell proliferation, down regulation of sebocyte proliferation, down-regulation of sebocyte proliferation, downregulation of sebocyte proliferation, inhibition of sebocyte proliferation, negative regulation of sebocyte proliferation Relationships: is a type of negative regulation of epithelial cell proliferation [GO:0050680]; is a type of regulation of sebum secreting cell proliferation [GO:1904002]; RO_0002212 GO:1990654